{
  "term_label": "nucleus",
  "gene_name": "Bcl-2-like protein 15",
  "term_id": "GO:0005634",
  "gene_symbol": "BCL2L15",
  "gene": "UniProtKB:Q5TBC7"
}